mitogen-activated protein kinase kinase kinase binding [GO:0031435] (molecular function) Relationships: is a type of protein kinase binding [GO:0019901] Definition: Binding to a mitogen-activated protein kinase kinase kinase, a protein that can phosphorylate a MAP kinase kinase. Also known as: MAPKKK binding Sources: GOC:bf